{
  "gene_symbol": "ODAD3",
  "term_label": "Unknown molecular function",
  "term_id": "UNKNOWN:0001",
  "gene": "UniProtKB:A5D8V7",
  "gene_name": "Outer dynein arm-docking complex subunit 3"
}